{
  "gene_name": "2'-5'-oligoadenylate synthase-like protein",
  "gene_symbol": "OASL",
  "term_id": "GO:0070106",
  "gene": "UniProtKB:Q15646",
  "term_label": "interleukin-27-mediated signaling pathway"
}